regulation of postsynaptic membrane neurotransmitter receptor levels [GO:0099072] (biological process) Subtypes: postsynaptic neurotransmitter receptor internalization [GO:0098884], exocytic insertion of neurotransmitter receptor to postsynaptic membrane [GO:0098967], GO:0098969, postsynaptic neurotransmitter receptor diffusion trapping [GO:0098970], neurotransmitter receptor localization to postsynaptic specialization membrane [GO:0099645] Sources: GOC:dos Relationships: is_a regulation of biological quality [GO:0065008] Definition: Any process that regulates the the local concentration of neurotransmitter receptor at the postsynaptic membrane.